{
  "gene_name": "MBT domain-containing protein 1",
  "gene": "UniProtKB:Q05BQ5",
  "term_id": "GO:0003682",
  "term_label": "chromatin binding",
  "gene_symbol": "MBTD1"
}